{
  "term_id": "GO:0006508",
  "term_label": "proteolysis",
  "gene_symbol": "ADAMTS3",
  "gene": "UniProtKB:O15072",
  "gene_name": "A disintegrin and metalloproteinase with thrombospondin motifs 3"
}